{
  "gene_symbol": "MT1H",
  "term_label": "cellular response to copper ion",
  "term_id": "GO:0071280",
  "gene": "UniProtKB:P80294",
  "gene_name": "Metallothionein-1H"
}